{
  "gene": "UniProtKB:Q9BYN0",
  "term_label": "cytoplasm",
  "gene_name": "Sulfiredoxin-1",
  "term_id": "GO:0005737",
  "gene_symbol": "SRXN1"
}